poly(ribitol-phosphate) N-acetylglucosaminyltransferase activity [GO:0047269] (molecular function) Sources: EC:2.4.1.70 Definition: Catalysis of the reaction: poly(ribitol phosphate) + UDP-N-acetyl-D-glucosamine = N-acetyl-D-glucosaminyl-poly(ribitol phosphate) + UDP. Relationships: is a type of acetylglucosaminyltransferase activity [GO:0008375] Also known as: UDP acetylglucosamine-poly(ribitol phosphate) acetylglucosaminyltransferase activity, UDP-N-acetyl-D-glucosamine:poly(ribitol-phosphate) N-acetyl-D-glucosaminyltransferase activity, uridine diphosphoacetylglucosamine-poly(ribitol phosphate) acetylglucosaminyltransferase activity